mechanosensitive potassium channel activity [GO:0098782] (molecular function) Relationships: is a type of GO:0005267; is a type of mechanosensitive monoatomic cation channel activity [GO:0140135] Definition: Enables the transmembrane transfer of a potassium ion by a channel that opens in response to a mechanical stress. References: PMID:22282805, PMID:25471887, PMID:25500157 Also known as: mechanically-gated potassium channel activity